{
  "gene_symbol": "ZP1",
  "gene": "UniProtKB:P60852",
  "gene_name": "Zona pellucida sperm-binding protein 1",
  "term_label": "structural constituent of egg coat",
  "term_id": "GO:0035804"
}